{
  "term_label": "endoplasmic reticulum-Golgi intermediate compartment",
  "gene": "UniProtKB:Q9Y3A6",
  "term_id": "GO:0005793",
  "gene_name": "Transmembrane emp24 domain-containing protein 5",
  "gene_symbol": "TMED5"
}